plasma lipoprotein particle clearance [GO:0034381] (biological process) Sources: GOC:BHF, GOC:ascb_2009, GOC:dph, GOC:mah, GOC:tb Also known as: lipoprotein particle clearance Subtypes: low-density lipoprotein particle clearance [GO:0034383], high-density lipoprotein particle clearance [GO:0034384], very-low-density lipoprotein particle clearance [GO:0034447], triglyceride-rich lipoprotein particle clearance [GO:0071830], oxidised low-density lipoprotein particle clearance [GO:0150024] Relationships: is a type of multicellular organismal process [GO:0032501]; is part of regulation of plasma lipoprotein particle levels [GO:0097006]; has part receptor-mediated endocytosis [GO:0006898]; has part plasma lipoprotein particle disassembly [GO:0071829] Definition: The process in which a lipoprotein particle is removed from the blood via receptor-mediated endocytosis and its constituent parts degraded. Regulation: regulated by regulation of lipoprotein particle clearance [GO:0010984]; negatively regulated by negative regulation of lipoprotein particle clearance [GO:0010985]; positively regulated by positive regulation of lipoprotein particle clearance [GO:0010986]